codeine metabolic process [GO:2001291] (biological process) Subtypes: GO:2001292 Also known as: codeine metabolism Sources: GOC:yaf Definition: The chemical reactions and pathways involving codeine, an alkaloid found in the opium poppy, Papaver somniferum var. album. Codeine has analgesic, anti-tussive and anti-diarrhoeal properties. Relationships: is a type of isoquinoline alkaloid metabolic process [GO:0033076]